thymidylate synthase (FAD) activity [GO:0050797] (molecular function) Relationships: is a type of 5,10-methylenetetrahydrofolate-dependent methyltransferase activity [GO:0042083] Also known as: Thy1 activity, ThyX activity, 5,10-methylenetetrahydrofolate,FADH2:dUMP C-methyltransferase activity, FDTS activity, flavin dependent thymidylate synthase activity Definition: Catalysis of the reaction: 5,10-methylenetetrahydrofolate + dUMP + NADPH + H+ = dTMP + tetrahydrofolate + NADP+. Sources: EC:2.1.1.148